{
  "term_label": "GTPase activity",
  "gene_name": "Septin-7",
  "gene_symbol": "SEPTIN7",
  "gene": "UniProtKB:Q16181",
  "term_id": "GO:0003924"
}